{
  "gene": "UniProtKB:Q8NDX2",
  "gene_symbol": "SLC17A8",
  "term_id": "GO:0050803",
  "gene_name": "Vesicular glutamate transporter 3",
  "term_label": "regulation of synapse structure or activity"
}